{
  "term_id": "UNKNOWN:0001",
  "gene_symbol": "HDGFL1",
  "gene": "UniProtKB:Q5TGJ6",
  "term_label": "Unknown molecular function",
  "gene_name": "Hepatoma-derived growth factor-like protein 1"
}